cerebellum vasculature morphogenesis [GO:0061301] (biological process) Definition: The process in which the vasculature of the cerebellum is generated and organized. Sources: GOC:BHF, GOC:dph Relationships: is a type of anatomical structure morphogenesis [GO:0009653]; is part of cerebellum development [GO:0021549]; is part of cerebellum vasculature development [GO:0061300]